{
  "gene": "UniProtKB:P04844",
  "term_label": "protein N-linked glycosylation",
  "gene_name": "Dolichyl-diphosphooligosaccharide--protein glycosyltransferase subunit 2",
  "gene_symbol": "RPN2",
  "term_id": "GO:0006487"
}